response to 11-deoxycorticosterone [GO:1903496] (biological process) Subtypes: cellular response to 11-deoxycorticosterone [GO:1903497] Relationships: is a type of response to mineralocorticoid [GO:0051385]; is a type of response to alcohol [GO:0097305]; is a type of response to ketone [GO:1901654] References: PMID:3585228 Sources: GOC:TermGenie, GOC:mr, GO_REF:0000071 Definition: Any process that results in a change in state or activity of a cell or an organism (in terms of movement, secretion, enzyme production, gene expression, etc.) as a result of a 11-deoxycorticosterone stimulus.